peripheral region of growth cone [GO:0090725] (cellular component) Definition: The non-central region or periphery of the migrating motile tip of a growing nerve cell axon or dendrite. References: PMID:16260607 Sources: GOC:sl Relationships: is a type of GO:0110165; is part of GO:0030426